{
  "gene_symbol": "DPYSL5",
  "term_label": "hydrolase activity, acting on carbon-nitrogen (but not peptide) bonds, in cyclic amides",
  "term_id": "GO:0016812",
  "gene_name": "Dihydropyrimidinase-related protein 5",
  "gene": "UniProtKB:Q9BPU6"
}